{
  "gene": "UniProtKB:Q96R27",
  "gene_symbol": "OR2M4",
  "term_label": "detection of chemical stimulus involved in sensory perception of smell",
  "term_id": "GO:0050911",
  "gene_name": "Olfactory receptor 2M4"
}